{
  "term_label": "extracellular space",
  "gene_symbol": "CCL5",
  "term_id": "GO:0005615",
  "gene": "UniProtKB:P13501",
  "gene_name": "C-C motif chemokine 5"
}